nonadec-1-ene metabolic process [GO:1900876] (biological process) Also known as: nonadec-1-ene metabolism Subtypes: nonadec-1-ene biosynthetic process [GO:1900877] Sources: GOC:TermGenie, GOC:mengo_curators Relationships: is a type of GO:1900673 Definition: The chemical reactions and pathways involving nonadec-1-ene.